{
  "gene": "UniProtKB:Q13442",
  "gene_symbol": "PDAP1",
  "gene_name": "28 kDa heat- and acid-stable phosphoprotein",
  "term_label": "cytosol",
  "term_id": "GO:0005829"
}